alkylamidase activity [GO:0047648] (molecular function) Relationships: is a type of hydrolase activity, acting on carbon-nitrogen (but not peptide) bonds, in linear amides [GO:0016811] Also known as: N-methylhexanamide amidohydrolase activity Sources: EC:3.5.1.39, RHEA:20081 Definition: Catalysis of the reaction: N-methylhexanamide + H2O = hexanoate + methylammonium.